7-beta-hydroxysteroid dehydrogenase (NADP+) activity [GO:0047022] (MF) Relationships: is a type of GO:0033764 Also known as: 7beta-hydroxysteroid dehydrogenase (NADP+), 7beta-hydroxysteroid:NADP+ 7-oxidoreductase activity, NADP-dependent 7-beta-hydroxysteroid dehydrogenase activity, NADP-dependent 7beta-hydroxysteroid dehydrogenase activity Definition: Catalysis of the reaction: a 7-beta-hydroxysteroid + NADP+ = a 7-oxosteroid + NADPH + H+. Sources: RHEA:20233